{
  "gene": "UniProtKB:Q16048",
  "gene_name": "Putative pro-MCH-like protein 1",
  "term_label": "negative regulation of synaptic transmission, dopaminergic",
  "gene_symbol": "PMCHL1",
  "term_id": "GO:0032227"
}